beta-adrenergic receptor activity [GO:0004939] (molecular function) Definition: Combining with epinephrine or norepinephrine to initiate a change in cell activity via activation of a G protein, with pharmacological characteristics of beta-adrenergic receptors; the activity involves transmitting the signal to the Gs alpha subunit of a heterotrimeric G protein. Relationships: is a type of adrenergic receptor activity [GO:0004935] Subtypes: beta1-adrenergic receptor activity [GO:0004940], beta2-adrenergic receptor activity [GO:0004941], beta3-adrenergic receptor activity [GO:0015052] Sources: GOC:cb, GOC:mah, IUPHAR_GPCR:1274 Also known as: beta adrenoceptor